{
  "term_label": "synaptic cleft",
  "gene": "UniProtKB:P55286",
  "gene_symbol": "CDH8",
  "term_id": "GO:0043083",
  "gene_name": "Cadherin-8"
}